{
  "gene": "UniProtKB:P02730",
  "term_label": "bicarbonate transmembrane transporter activity",
  "term_id": "GO:0015106",
  "gene_symbol": "SLC4A1",
  "gene_name": "Band 3 anion transport protein"
}